{
  "term_id": "UNKNOWN:0001",
  "gene_name": "Ankyrin repeat and SAM domain-containing protein 4B",
  "gene_symbol": "ANKS4B",
  "term_label": "Unknown molecular function",
  "gene": "UniProtKB:Q8N8V4"
}